{
  "gene_name": "Leukocyte-associated immunoglobulin-like receptor 1",
  "gene": "UniProtKB:Q6GTX8",
  "term_id": "GO:0004888",
  "gene_symbol": "LAIR1",
  "term_label": "transmembrane signaling receptor activity"
}